{
  "term_id": "GO:0005634",
  "gene_symbol": "ZNF384",
  "gene_name": "Zinc finger protein 384",
  "gene": "UniProtKB:Q8TF68",
  "term_label": "nucleus"
}